{
  "gene_symbol": "ITSN1",
  "gene_name": "Intersectin-1",
  "term_id": "GO:0005737",
  "term_label": "cytoplasm",
  "gene": "UniProtKB:Q15811"
}